endo-1,3-alpha-L-rhamnosidase activity [GO:0052775] (molecular function) Definition: Catalysis of the reaction: R1-L-rhamnose-(1->3)-alpha-L-rhamnose-R2 + H2O = R1-L-rhamnose + L-rhamnose-R2. This reaction is the hydrolysis of an alpha-(1->3) linkage between two rhamnose residues in a polysaccharide chain. Also known as: endorhamnosidase activity, endo-(1,3)-alpha-L-rhamnosidase activity, endo-(1->3)-alpha-L-rhamnosidase activity References: PMID:10439404 Sources: GOC:mengo_curators Relationships: is a type of hydrolase activity, hydrolyzing O-glycosyl compounds [GO:0004553]